{
  "gene_symbol": "MARK3",
  "term_label": "tau-protein kinase activity",
  "term_id": "GO:0050321",
  "gene_name": "MAP_microtubule affinity-regulating kinase 3",
  "gene": "UniProtKB:P27448"
}